{
  "gene_name": "PRAME family member 22",
  "term_label": "cytoplasm",
  "gene_symbol": "PRAMEF22",
  "gene": "UniProtKB:A3QJZ6",
  "term_id": "GO:0005737"
}